{
  "term_label": "neuron projection",
  "term_id": "GO:0043005",
  "gene_symbol": "CHRNB3",
  "gene": "UniProtKB:Q05901",
  "gene_name": "Neuronal acetylcholine receptor subunit beta-3"
}